{
  "gene_symbol": "TMEM86A",
  "term_label": "Unknown biological process",
  "gene": "UniProtKB:Q8N2M4",
  "term_id": "UNKNOWN:0002",
  "gene_name": "Lysoplasmalogenase-like protein TMEM86A"
}